symbiont-mediated activation of host MAPK cascade [GO:0141071] (biological process) Relationships: is_a symbiont-mediated activation of host signal transduction pathway [GO:0052028]; is_a symbiont-mediated perturbation of host MAPK cascade [GO:0052080] References: PMID:24043761, PMID:25675415, PMID:28166272 Definition: A process in which a symbiont subverts a MAPK signal transduction pathway in the host organism by initiating, promoting, or enhancing its activation. The host is defined as the larger of the organisms involved in a symbiotic interaction. Also known as: induction by symbiont of host MAP kinase signal transduction pathway, induction of host MAPK kinase signaling pathway, symbiont-mediated activation of host MAPK signal transduction pathway, activation by symbiont of host MAPK signal transduction pathway, stimulation by symbiont of host MAPK signal transduction pathway